calcium ion sensor activity [GO:0061891] (molecular function) Relationships: is a type of metal ion sensor activity [GO:0140784]; has part calcium ion binding [GO:0005509] Definition: Binding to and responding, e.g. by conformational change, to changes in the cellular level of calcium ions (Ca2+). References: PMID:16005298, PMID:17020874, PMID:28151650